{
  "gene_name": "Olfactory receptor 8U1",
  "term_label": "Unknown biological process",
  "gene": "UniProtKB:Q8NH10",
  "gene_symbol": "OR8U1",
  "term_id": "UNKNOWN:0002"
}